{
  "term_id": "GO:0035332",
  "gene": "UniProtKB:P0DPB3",
  "term_label": "positive regulation of hippo signaling",
  "gene_name": "Schwannomin-interacting protein 1",
  "gene_symbol": "SCHIP1"
}